negative regulation of response to gamma radiation [GO:2001229] (biological process) Definition: Any process that stops, prevents or reduces the frequency, rate or extent of response to gamma radiation. Sources: GOC:obol Also known as: negative regulation of response to gamma ray, negative regulation of response to gamma-ray photon Relationships: is_a negative regulation of response to stimulus [GO:0048585]; is a type of regulation of response to gamma radiation [GO:2001228]; negatively regulates response to gamma radiation [GO:0010332] Subtypes: negative regulation of cellular response to gamma radiation [GO:1905844]